{
  "term_label": "Unknown molecular function",
  "term_id": "UNKNOWN:0001",
  "gene": "UniProtKB:P15502",
  "gene_name": "Elastin",
  "gene_symbol": "ELN"
}